{
  "gene_symbol": "RND3",
  "gene": "UniProtKB:P61587",
  "gene_name": "Rho-related GTP-binding protein RhoE",
  "term_id": "GO:0032956",
  "term_label": "regulation of actin cytoskeleton organization"
}